{
  "gene_name": "Oxytocin receptor",
  "term_label": "cellular response to hormone stimulus",
  "term_id": "GO:0032870",
  "gene_symbol": "OXTR",
  "gene": "UniProtKB:P30559"
}